fungal-type cell wall disassembly involved in conjugation with cellular fusion [GO:1904541] (biological process) References: PMID:25825517 Sources: GOC:TermGenie, GO_REF:0000060 Relationships: is a type of cell wall organization involved in conjugation with cellular fusion [GO:0070871]; is_a fungal-type cell wall disassembly [GO:0071853] Also known as: fungal-type cell wall disassembly involved in cell fusion, fungal-type cell wall disassembly involved in mating Definition: Any fungal-type cell wall disassembly that is involved in conjugation with cellular fusion.